{
  "gene_name": "Membrane primary amine oxidase",
  "term_label": "amine metabolic process",
  "gene": "UniProtKB:Q16853",
  "term_id": "GO:0009308",
  "gene_symbol": "AOC3"
}